{
  "gene_symbol": "LAMP3",
  "gene": "UniProtKB:Q9UQV4",
  "term_label": "lysosomal membrane",
  "term_id": "GO:0005765",
  "gene_name": "Lysosome-associated membrane glycoprotein 3"
}